11-cis-retinol dehydrogenase (NADP+) activity [GO:0102354] (molecular function) Also known as: 11-cis-retinol dehydrogenase activity Sources: RHEA:54912 Definition: Catalysis of the reaction: 11-cis-retinol + NADP+ = 11-cis-retinal + NADPH + H+. Relationships: is_a GO:0008106